{
  "term_id": "GO:0007095",
  "gene_name": "Denticleless protein homolog",
  "term_label": "mitotic G2 DNA damage checkpoint signaling",
  "gene_symbol": "DTL",
  "gene": "UniProtKB:Q9NZJ0"
}